{
  "term_label": "positive regulation of transcription by RNA polymerase II",
  "gene_symbol": "VDR",
  "gene_name": "Vitamin D3 receptor",
  "term_id": "GO:0045944",
  "gene": "UniProtKB:P11473"
}